{
  "gene_name": "Alpha-2-HS-glycoprotein",
  "gene_symbol": "AHSG",
  "gene": "UniProtKB:P02765",
  "term_id": "GO:0031012",
  "term_label": "extracellular matrix"
}